succinyl-CoA biosynthetic process [GO:1901290] (BP) Subtypes: 2-oxoglutarate decarboxylation to succinyl-CoA [GO:0120551] Definition: The chemical reactions and pathways resulting in the formation of succinyl-CoA. Also known as: succinyl-CoA anabolism, succinyl-CoA biosynthesis, succinyl-CoA formation, succinyl-CoA synthesis Relationships: is a type of succinyl-CoA metabolic process [GO:0006104]; is a type of acyl-CoA biosynthetic process [GO:0071616] Sources: GOC:TermGenie, GOC:yaf, UniPathway:UPA00929